lumen formation, open tracheal system [GO:0035149] (biological process) Definition: Creation of the central hole of a tube in an open tracheal system through which gases flow. Relationships: is_a GO:0035148; is a type of regulation of tube architecture, open tracheal system [GO:0035152] Also known as: tracheal lumen formation Sources: GOC:bf, GOC:mtg_sensu